nicotinate-O-glucosyltransferase activity [GO:0090704] (molecular function) Relationships: is a type of UDP-glucosyltransferase activity [GO:0035251] Definition: Catalysis of the reaction: nicotinate + UDP-D-glucose = O-D-glucosylnicotinate + UDP. References: PMID:26116607 Sources: GOC:tb